{
  "term_id": "UNKNOWN:0002",
  "gene_symbol": "SPACA9",
  "term_label": "Unknown biological process",
  "gene": "UniProtKB:Q96E40",
  "gene_name": "Sperm acrosome-associated protein 9"
}